{
  "term_label": "extracellular space",
  "term_id": "GO:0005615",
  "gene_name": "Fibroblast growth factor 6",
  "gene_symbol": "FGF6",
  "gene": "UniProtKB:P10767"
}